{
  "gene_name": "Potassium voltage-gated channel subfamily S member 2",
  "gene": "UniProtKB:Q9ULS6",
  "term_label": "action potential",
  "gene_symbol": "KCNS2",
  "term_id": "GO:0001508"
}